guanine transmembrane transport [GO:1903716] (biological process) Relationships: is a type of guanine transport [GO:0015854]; is a type of purine nucleobase transmembrane transport [GO:1904823] Definition: The process in which guanine is transported across a membrane. Subtypes: guanine import across plasma membrane [GO:0098710], mitochondrial guanine nucleotide transmembrane transport [GO:0140140] References: PMID:14998997 Sources: GOC:TermGenie, GO_REF:0000069